symbiont-mediated cytolysis of host cell [GO:0001897] (biological process) Definition: A process mediated by a symbiont that results in the death of a host cell by means of the rupture of cell membranes and the loss of cytoplasm. The host is defined as the larger of the organisms involved in a symbiotic interaction. References: PMID:11423190, PMID:23748204, PMID:24204713, PMID:27405240 Subtypes: GO:0019836, viral release from host cell by cytolysis [GO:0044659] Also known as: cytolysis by organism of host cells, cytolysis by symbiont of host cells, pathogenesis Relationships: is a type of symbiont-mediated killing of host cell [GO:0001907]; is a type of GO:0051715